{
  "gene_symbol": "C1RL",
  "term_id": "GO:0004252",
  "gene": "UniProtKB:Q9NZP8",
  "term_label": "serine-type endopeptidase activity",
  "gene_name": "Complement C1r subcomponent-like protein"
}